{
  "term_label": "Unknown molecular function",
  "gene_name": "Protein BANP",
  "gene_symbol": "BANP",
  "term_id": "UNKNOWN:0001",
  "gene": "UniProtKB:Q8N9N5"
}